negative regulation of blood vessel endothelial cell proliferation involved in sprouting angiogenesis [GO:1903588] (biological process) References: PMID:23388056 Sources: GOC:TermGenie, GO_REF:0000058 Relationships: is a type of negative regulation of endothelial cell proliferation [GO:0001937]; is a type of regulation of blood vessel endothelial cell proliferation involved in sprouting angiogenesis [GO:1903587]; negatively regulates GO:0002043 Definition: Any process that stops, prevents or reduces the frequency, rate or extent of blood vessel endothelial cell proliferation involved in sprouting angiogenesis. Also known as: down regulation of blood vessel endothelial cell proliferation involved in sprouting angiogenesis, down-regulation of blood vessel endothelial cell proliferation involved in sprouting angiogenesis, downregulation of blood vessel endothelial cell proliferation involved in sprouting angiogenesis, inhibition of blood vessel endothelial cell proliferation involved in sprouting angiogenesis, down regulation of blood vessel endothelial cell proliferation during sprouting angiogenesis, down-regulation of blood vessel endothelial cell proliferation during sprouting angiogenesis, downregulation of blood vessel endothelial cell proliferation during sprouting angiogenesis, inhibition of blood vessel endothelial cell proliferation during sprouting angiogenesis, negative regulation of blood vessel endothelial cell proliferation during sprouting angiogenesis